{
  "term_label": "Unknown biological process",
  "gene_symbol": "TATDN1",
  "gene": "UniProtKB:Q6P1N9",
  "gene_name": "Deoxyribonuclease TATDN1",
  "term_id": "UNKNOWN:0002"
}